initiation of neural tube closure [GO:0021993] (BP) Relationships: is a type of GO:0002009; is a type of embryonic morphogenesis [GO:0048598]; is part of neural tube closure [GO:0001843] Definition: The process in which closure points are established at multiple points and along the neural rostrocaudal axis. Sources: GOC:cls, GOC:dgh, GOC:dph, GOC:jid, GO_REF:0000021